phosphatidylcholine transporter activity [GO:0008525] (molecular function) Also known as: phosphatidylcholine transmembrane transporter activity Sources: GOC:ai, ISBN:0198506732 Definition: Enables the directed movement of phosphatidylcholine into, out of or within a cell, or between cells. Phosphatidylcholine refers to a class of glycerophospholipids in which the phosphatidyl group is esterified to the hydroxyl group of choline. Subtypes: phosphatidylcholine floppase activity [GO:0090554], phosphatidylcholine transfer activity [GO:0120019], phosphatidylcholine flippase activity [GO:0140345] Relationships: is a type of GO:0005548